{
  "gene": "UniProtKB:Q502X0",
  "term_id": "UNKNOWN:0002",
  "gene_name": "MORN repeat-containing protein 2",
  "gene_symbol": "MORN2",
  "term_label": "Unknown biological process"
}